{
  "gene_name": "Tissue factor pathway inhibitor",
  "term_id": "GO:0005615",
  "term_label": "extracellular space",
  "gene_symbol": "TFPI",
  "gene": "UniProtKB:P10646"
}